{
  "term_label": "hepatocyte growth factor receptor binding",
  "gene_symbol": "ESM1",
  "gene_name": "Endothelial cell-specific molecule 1",
  "term_id": "GO:0005171",
  "gene": "UniProtKB:Q9NQ30"
}